{
  "term_label": "transcription cis-regulatory region binding",
  "term_id": "GO:0000976",
  "gene": "UniProtKB:Q8TF68",
  "gene_name": "Zinc finger protein 384",
  "gene_symbol": "ZNF384"
}